{
  "gene": "UniProtKB:Q8N3A8",
  "term_id": "GO:0043539",
  "gene_name": "Protein mono-ADP-ribosyltransferase PARP8",
  "gene_symbol": "PARP8",
  "term_label": "protein serine/threonine kinase activator activity"
}